{
  "gene_name": "D-amino-acid oxidase",
  "gene_symbol": "DAO",
  "term_label": "D-amino-acid oxidase activity",
  "gene": "UniProtKB:P14920",
  "term_id": "GO:0003884"
}